{
  "gene_symbol": "GNAQ",
  "gene": "UniProtKB:P50148",
  "term_id": "GO:0003924",
  "gene_name": "Guanine nucleotide-binding protein G(q) subunit alpha",
  "term_label": "GTPase activity"
}